regulation of cell cycle G2/M phase transition [GO:1902749] (biological process) Sources: GOC:TermGenie, GOC:jl, GO_REF:0000058 Definition: Any signaling pathway that modulates the activity of a cell cycle cyclin-dependent protein kinase to modulate the switch from G2 phase to M phase of the cell cycle. Subtypes: regulation of G2/M transition of mitotic cell cycle [GO:0010389], regulation of G2/MI transition of meiotic cell cycle [GO:0110030], negative regulation of cell cycle G2/M phase transition [GO:1902750], positive regulation of cell cycle G2/M phase transition [GO:1902751] Relationships: is a type of regulation of cell cycle phase transition [GO:1901987]; regulates GO:0044839